{
  "gene_name": "Elongation of very long chain fatty acids protein 6",
  "term_label": "fatty acid elongase activity",
  "gene_symbol": "ELOVL6",
  "term_id": "GO:0009922",
  "gene": "UniProtKB:Q9H5J4"
}